{
  "gene": "UniProtKB:P10911",
  "gene_symbol": "MCF2",
  "term_label": "guanyl-nucleotide exchange factor activity",
  "gene_name": "Proto-oncogene DBL",
  "term_id": "GO:0005085"
}